{
  "term_id": "GO:0012506",
  "gene": "UniProtKB:P20073",
  "term_label": "vesicle membrane",
  "gene_name": "Annexin A7",
  "gene_symbol": "ANXA7"
}